{
  "gene": "UniProtKB:P16870",
  "gene_symbol": "CPE",
  "term_label": "metallocarboxypeptidase activity",
  "gene_name": "Carboxypeptidase E",
  "term_id": "GO:0004181"
}